{
  "term_id": "GO:0031012",
  "gene_name": "Extracellular matrix protein 2",
  "term_label": "extracellular matrix",
  "gene": "UniProtKB:O94769",
  "gene_symbol": "ECM2"
}